{
  "gene_symbol": "DHX57",
  "term_id": "UNKNOWN:0002",
  "gene": "UniProtKB:Q6P158",
  "term_label": "Unknown biological process",
  "gene_name": "Putative ATP-dependent RNA helicase DHX57"
}